{
  "gene_name": "AP-3 complex subunit delta-1",
  "gene": "UniProtKB:O14617",
  "term_label": "Golgi to vacuole transport",
  "gene_symbol": "AP3D1",
  "term_id": "GO:0006896"
}